{
  "gene_symbol": "GALNT2",
  "gene_name": "Polypeptide N-acetylgalactosaminyltransferase 2",
  "term_id": "GO:0004653",
  "gene": "UniProtKB:Q10471",
  "term_label": "polypeptide N-acetylgalactosaminyltransferase activity"
}